{
  "gene_name": "Acid sphingomyelinase-like phosphodiesterase 3a",
  "gene": "UniProtKB:Q92484",
  "gene_symbol": "SMPDL3A",
  "term_id": "UNKNOWN:0002",
  "term_label": "Unknown biological process"
}